{
  "gene": "UniProtKB:Q06495",
  "gene_name": "Sodium-dependent phosphate transport protein 2A",
  "term_label": "vesicle",
  "term_id": "GO:0031982",
  "gene_symbol": "SLC34A1"
}